{
  "term_label": "transmembrane signaling receptor activity",
  "gene_symbol": "FCRL5",
  "gene": "UniProtKB:Q96RD9",
  "term_id": "GO:0004888",
  "gene_name": "Fc receptor-like protein 5"
}